{
  "term_id": "GO:0015908",
  "term_label": "fatty acid transport",
  "gene_name": "Cellular retinoic acid-binding protein 2",
  "gene_symbol": "CRABP2",
  "gene": "UniProtKB:P29373"
}